{
  "gene": "UniProtKB:P0C7P1",
  "gene_name": "RNA-binding motif protein, Y chromosome, family 1 member D",
  "gene_symbol": "RBMY1D",
  "term_id": "GO:0000398",
  "term_label": "mRNA splicing, via spliceosome"
}